response to phorbol 13-acetate 12-myristate [GO:1904627] (biological process) References: PMID:2200903 Sources: GOC:TermGenie, GO_REF:0000071 Also known as: response to PMA, response to TPA, response to phorbol 12-tetradecanoate 13-acetate, response to tetradecanoylphorbol acetate Subtypes: cellular response to phorbol 13-acetate 12-myristate [GO:1904628] Relationships: is a type of response to lipid [GO:0033993]; is a type of response to alcohol [GO:0097305]; is a type of GO:1901654 Definition: Any process that results in a change in state or activity of a cell or an organism (in terms of movement, secretion, enzyme production, gene expression, etc.) as a result of a phorbol 13-acetate 12-myristate stimulus.